{
  "term_label": "Unknown molecular function",
  "gene": "UniProtKB:Q96MD7",
  "gene_symbol": "C9orf85",
  "gene_name": "Uncharacterized protein C9orf85",
  "term_id": "UNKNOWN:0001"
}